negative regulation of acylglycerol transport [GO:1901507] (biological process) Sources: GOC:TermGenie, GOC:sart Subtypes: negative regulation of triglyceride transport [GO:1905884] Relationships: is_a negative regulation of lipid transport [GO:0032369]; is a type of regulation of acylglycerol transport [GO:1901506]; RO_0002212 GO:0034196 Also known as: down regulation of acylglycerol transport, down regulation of glyceride transport, down-regulation of acylglycerol transport, down-regulation of glyceride transport, downregulation of acylglycerol transport, downregulation of glyceride transport, negative regulation of glyceride transport, inhibition of acylglycerol transport, inhibition of glyceride transport Definition: Any process that stops, prevents or reduces the frequency, rate or extent of acylglycerol transport.